{
  "gene": "UniProtKB:O14646",
  "gene_name": "Chromodomain-helicase-DNA-binding protein 1",
  "term_id": "GO:0003682",
  "gene_symbol": "CHD1",
  "term_label": "chromatin binding"
}